{
  "term_label": "Unknown molecular function",
  "gene_symbol": "TRBV11-2",
  "gene_name": "T cell receptor beta variable 11-2",
  "term_id": "UNKNOWN:0001",
  "gene": "UniProtKB:A0A584"
}